diamine oxidase activity [GO:0052597] (molecular function) Relationships: is a type of oxidoreductase activity, acting on the CH-NH2 group of donors, oxygen as acceptor [GO:0016641] Definition: Catalysis of the reaction: a diamine + H2O + O2 = a monoamine + NH4+ + H2O2. Also known as: diamine:oxygen oxidoreductase (deaminating) activity Subtypes: protein-lysine 6-oxidase activity [GO:0004720], putrescine oxidase activity [GO:0050232], histamine oxidase activity [GO:0052598] Sources: MetaCyc:RXN-9599